{
  "gene_symbol": "MORN3",
  "term_label": "Unknown cellular component",
  "term_id": "UNKNOWN:0003",
  "gene_name": "MORN repeat-containing protein 3",
  "gene": "UniProtKB:Q6PF18"
}